MATH domain binding [GO:0090736] (molecular function) Relationships: is a type of protein domain specific binding [GO:0019904] References: PMID:22621901 Sources: InterPro:IPR002083 Definition: Binding to a meprin and TRAF homology (MATH) domain.